positive regulation of chromosome attachment to the nuclear envelope [GO:0120266] (biological process) Relationships: is a type of GO:0090068; is a type of regulation of chromosome attachment to the nuclear envelope [GO:0120264]; positively regulates chromosome attachment to the nuclear envelope [GO:0097240] Sources: GOC:krc Also known as: up regulation of chromosome attachment to the nuclear envelope, up-regulation of chromosome attachment to the nuclear envelope, upregulation of chromosome attachment to the nuclear envelope, activation of chromosome attachment to the nuclear envelope, stimulation of chromosome attachment to the nuclear envelope Definition: Any process that activates or increases the frequency, rate or extent of the chromosome attachment to the nuclear envelope.